{
  "gene_name": "Putative uncharacterized protein ERCC6L2-AS1",
  "gene": "UniProtKB:Q8WZB0",
  "term_id": "UNKNOWN:0002",
  "term_label": "Unknown biological process",
  "gene_symbol": "ERCC6L2-AS1"
}